{
  "term_id": "UNKNOWN:0001",
  "gene_name": "Transmembrane protein 253",
  "gene_symbol": "TMEM253",
  "gene": "UniProtKB:P0C7T8",
  "term_label": "Unknown molecular function"
}